{
  "gene": "UniProtKB:P12109",
  "term_label": "skeletal muscle fiber development",
  "gene_symbol": "COL6A1",
  "term_id": "GO:0048741",
  "gene_name": "Collagen alpha-1(VI) chain"
}